{
  "term_id": "GO:0005615",
  "gene_name": "C-C motif chemokine 13",
  "term_label": "extracellular space",
  "gene": "UniProtKB:Q99616",
  "gene_symbol": "CCL13"
}